{
  "term_label": "cytoplasmic vesicle",
  "gene_name": "Guanylate-binding protein 6",
  "gene": "UniProtKB:Q6ZN66",
  "gene_symbol": "GBP6",
  "term_id": "GO:0031410"
}